cholate 12-alpha dehydrogenase (NADP+) activity [GO:0047013] (molecular function) Relationships: is_a steroid dehydrogenase activity, acting on the CH-OH group of donors, NAD or NADP as acceptor [GO:0033764] Also known as: 12-alpha-hydroxysteroid dehydrogenase activity, 12alpha-hydroxy steroid dehydrogenase activity, 12alpha-hydroxysteroid dehydrogenase activity, 12alpha-hydroxysteroid:NADP+ 12-oxidoreductase activity, NAD-dependent 12alpha-hydroxysteroid dehydrogenase activity, NADP-12alpha-hydroxysteroid dehydrogenase activity Definition: Catalysis of the reaction: cholate + NADP+ = 3-alpha,7-alpha-dihydroxy-12-oxo-5-beta-cholanate + H+ + NADPH. Sources: RHEA:14129